{
  "term_label": "regulation of transcription by RNA polymerase II",
  "term_id": "GO:0006357",
  "gene_symbol": "DMRTA2",
  "gene_name": "Doublesex- and mab-3-related transcription factor A2",
  "gene": "UniProtKB:Q96SC8"
}